{
  "term_label": "adenylate cyclase inhibiting G protein-coupled glutamate receptor activity",
  "gene_symbol": "GRM1",
  "term_id": "GO:0001640",
  "gene_name": "Metabotropic glutamate receptor 1",
  "gene": "UniProtKB:Q13255"
}